{
  "gene_symbol": "ELOVL3",
  "gene_name": "Elongation of very long chain fatty acids protein 3",
  "gene": "UniProtKB:Q9HB03",
  "term_id": "GO:0030148",
  "term_label": "sphingolipid biosynthetic process"
}